ADP biosynthetic process [GO:0006172] (biological process) Definition: The chemical reactions and pathways resulting in the formation of ADP, adenosine 5'-diphosphate. Sources: GOC:ai Relationships: is a type of purine ribonucleotide biosynthetic process [GO:0009152]; is a type of purine ribonucleoside diphosphate biosynthetic process [GO:0009180]; is a type of ADP metabolic process [GO:0046031] Also known as: ADP anabolism, ADP biosynthesis, ADP formation, ADP synthesis